{
  "gene_symbol": "PAN2",
  "gene_name": "PAN2-PAN3 deadenylation complex catalytic subunit PAN2",
  "gene": "UniProtKB:Q504Q3",
  "term_label": "PAN complex",
  "term_id": "GO:0031251"
}